{
  "gene": "UniProtKB:Q9H6I2",
  "gene_name": "Transcription factor SOX-17",
  "term_label": "negative regulation of canonical Wnt signaling pathway",
  "gene_symbol": "SOX17",
  "term_id": "GO:0090090"
}